{
  "gene_name": "Inhibitory synaptic factor 2A",
  "term_label": "postsynaptic density",
  "gene": "UniProtKB:Q6ZSG2",
  "term_id": "GO:0014069",
  "gene_symbol": "INSYN2A"
}